{
  "gene_symbol": "NINJ1",
  "term_id": "GO:0019835",
  "gene": "UniProtKB:Q92982",
  "gene_name": "Ninjurin-1",
  "term_label": "cytolysis"
}